fatty acid O-methyltransferase activity [GO:0030733] (molecular function) Also known as: fatty-acid O-methyltransferase activity, S-adenosyl-L-methionine:fatty-acid O-methyltransferase activity, fatty acid methyltransferase activity Sources: EC:2.1.1.15 Definition: Catalysis of the reaction: S-adenosyl-L-methionine + a fatty acid = S-adenosyl-L-homocysteine + a fatty acid methyl ester. Relationships: is a type of S-adenosylmethionine-dependent methyltransferase activity [GO:0008757]